{
  "gene_name": "Meteorin-like protein",
  "gene_symbol": "METRNL",
  "gene": "UniProtKB:Q641Q3",
  "term_label": "hormone activity",
  "term_id": "GO:0005179"
}